transcription cis-regulatory region binding [GO:0000976] (molecular function) Definition: Binding to a specific sequence of DNA that is part of a regulatory region that controls transcription of that section of the DNA. The transcribed region might be described as a gene, cistron, or operon. Sources: GOC:txnOH Also known as: regulatory region DNA binding, transcription regulatory region sequence-specific DNA binding, bacterial-type RNA polymerase regulatory region DNA binding, bacterial-type RNA polymerase transcription regulatory region sequence-specific DNA binding, eubacterial-type RNA polymerase regulatory region DNA binding, eubacterial-type RNA polymerase regulatory region sequence-specific DNA binding, transcription regulatory region DNA binding Note: Note that this term is meant to also capture non-specific binding to regulatory regions. Also, to minimize ambiguity in the use of the word "promoter" in GO, we have chosen the phrase "transcription regulatory region" to refer to all of the regulatory regions. Regulatory regions in the DNA which control initiation may include the "core promoter" where the basal transcription machinery binds, the "core promoter proximal region" where regulatory factors other than the basal machinery bind. There are also additional regulatory regions, in both the DNA and the RNA transcript, which regulate elongation or termination of transcription. Relationships: is a type of GO:0001067; is a type of GO:1990837 Subtypes: RNA polymerase II transcription regulatory region sequence-specific DNA binding [GO:0000977], cis-regulatory region sequence-specific DNA binding [GO:0000987], GO:0001016, mitochondrial promoter sequence-specific DNA binding [GO:0001018], GO:0001019, core promoter sequence-specific DNA binding [GO:0001046], GO:0001147, intronic transcription regulatory region sequence-specific DNA binding [GO:0001161], RNA polymerase I transcription regulatory region sequence-specific DNA binding [GO:0001163], purine-rich negative regulatory element binding [GO:0032422] Regulation: regulated by GO:2000677; negatively regulated by negative regulation of transcription regulatory region DNA binding [GO:2000678]; RO_0002213 by positive regulation of transcription regulatory region DNA binding [GO:2000679]